{
  "term_label": "DNA-binding transcription factor activity, RNA polymerase II-specific",
  "term_id": "GO:0000981",
  "gene_name": "Double homeobox protein 4",
  "gene_symbol": "DUX4",
  "gene": "UniProtKB:Q9UBX2"
}